{
  "gene_name": "Serine protease 33",
  "term_id": "GO:0006508",
  "term_label": "proteolysis",
  "gene": "UniProtKB:Q8NF86",
  "gene_symbol": "PRSS33"
}